{
  "term_id": "GO:0005085",
  "gene_name": "Protein DENND6A",
  "term_label": "guanyl-nucleotide exchange factor activity",
  "gene": "UniProtKB:Q8IWF6",
  "gene_symbol": "DENND6A"
}